{
  "term_id": "GO:0007005",
  "gene_name": "Lon protease homolog, mitochondrial",
  "gene_symbol": "LONP1",
  "gene": "UniProtKB:P36776",
  "term_label": "mitochondrion organization"
}